negative regulation of RNA-dependent RNA polymerase activity [GO:1900260] (biological process) Definition: Any process that stops, prevents or reduces the frequency, rate or extent of RNA-directed 5'-3' RNA polymerase activity. Also known as: down regulation of transcriptase, down-regulation of transcriptase, downregulation of transcriptase, inhibition of transcriptase, negative regulation of RNA-directed RNA polymerase activity, negative regulation of transcriptase, down regulation of RNA nucleotidyltransferase (RNA-directed) activity, down regulation of RNA replicase activity, down regulation of RNA-dependent RNA polymerase activity, down regulation of RNA-dependent RNA replicase activity, down regulation of RNA-dependent ribonucleate nucleotidyltransferase activity, down regulation of RNA-directed RNA polymerase activity, down regulation of ribonucleic acid replicase activity, down regulation of ribonucleic acid-dependent ribonucleate nucleotidyltransferase activity, down regulation of ribonucleic acid-dependent ribonucleic acid polymerase activity, down regulation of ribonucleic replicase activity, down-regulation of RNA nucleotidyltransferase (RNA-directed) activity, down-regulation of RNA replicase activity, down-regulation of RNA-dependent RNA polymerase activity, down-regulation of RNA-dependent RNA replicase activity, down-regulation of RNA-dependent ribonucleate nucleotidyltransferase activity, down-regulation of RNA-directed RNA polymerase activity, down-regulation of ribonucleic acid replicase activity, downregulation of RNA nucleotidyltransferase (RNA-directed) activity, downregulation of RNA replicase activity, downregulation of RNA-dependent RNA polymerase activity, downregulation of RNA-dependent RNA replicase activity, downregulation of RNA-dependent ribonucleate nucleotidyltransferase activity, downregulation of RNA-directed RNA polymerase activity, downregulation of nucleoside-triphosphate:RNA nucleotidyltransferase (RNA-directed), downregulation of ribonucleic acid replicase activity, downregulation of ribonucleic acid-dependent ribonucleate nucleotidyltransferase activity, downregulation of ribonucleic acid-dependent ribonucleic acid polymerase activity, downregulation of ribonucleic replicase activity, inhibition of RNA nucleotidyltransferase (RNA-directed) activity, inhibition of RNA replicase activity, inhibition of RNA-dependent RNA polymerase activity, inhibition of RNA-dependent RNA replicase activity, inhibition of RNA-dependent ribonucleate nucleotidyltransferase activity, inhibition of nucleoside-triphosphate:RNA nucleotidyltransferase (RNA-directed), inhibition of ribonucleic acid replicase activity, inhibition of ribonucleic acid-dependent ribonucleate nucleotidyltransferase activity, inhibition of ribonucleic acid-dependent ribonucleic acid polymerase activity, inhibition of ribonucleic replicase activity, negative regulation of 3D polymerase activity, negative regulation of RNA nucleotidyltransferase (RNA-directed) activity, negative regulation of RNA replicase activity, negative regulation of RNA-dependent RNA replicase activity, negative regulation of RNA-dependent ribonucleate nucleotidyltransferase activity, negative regulation of RNA-directed 5'-3' RNA polymerase activity, negative regulation of nucleoside-triphosphate:RNA nucleotidyltransferase (RNA-directed), negative regulation of ribonucleic acid replicase activity, negative regulation of ribonucleic acid-dependent ribonucleate nucleotidyltransferase activity, negative regulation of ribonucleic acid-dependent ribonucleic acid polymerase activity, negative regulation of ribonucleic replicase activity, down regulation of phage f2 replicase, down-regulation of phage f2 replicase, downregulation of phage f2 replicase, inhibition of RNA-directed RNA polymerase activity, inhibition of phage f2 replicase, negative regulation of phage f2 replicase, down regulation of PB1 proteins, down regulation of PB2 proteins, down regulation of RDRP, down regulation of RNA synthetase activity, down regulation of polymerase L, down regulation of ribonucleic synthetase activity, down-regulation of PB1 proteins, down-regulation of PB2 proteins, down-regulation of RDRP, down-regulation of RNA synthetase activity, down-regulation of polymerase L, down-regulation of ribonucleic synthetase activity, downregulation of PB1 proteins, downregulation of PB2 proteins, downregulation of RDRP, downregulation of RNA synthetase activity, downregulation of polymerase L, downregulation of ribonucleic synthetase activity, inhibition of PB1 proteins, inhibition of PB2 proteins, inhibition of RDRP, inhibition of RNA synthetase activity, inhibition of polymerase L, inhibition of ribonucleic synthetase activity, negative regulation of PB1 proteins, negative regulation of PB2 proteins, negative regulation of RDRP, negative regulation of RNA synthetase activity, negative regulation of polymerase L, negative regulation of ribonucleic synthetase activity Sources: GOC:TermGenie, GOC:pf Relationships: is a type of negative regulation of catalytic activity [GO:0043086]; is a type of regulation of transferase activity [GO:0051338]; negatively regulates RNA-directed RNA polymerase activity [GO:0003968]